{
  "term_id": "GO:0005315",
  "term_label": "phosphate transmembrane transporter activity",
  "gene_name": "Solute carrier family 25 member 3",
  "gene": "UniProtKB:Q00325",
  "gene_symbol": "SLC25A3"
}